{
  "term_label": "Unknown molecular function",
  "gene": "UniProtKB:F8WBI6",
  "gene_symbol": "GOLGA8N",
  "term_id": "UNKNOWN:0001",
  "gene_name": "Golgin subfamily A member 8N"
}